cardiac right ventricle morphogenesis [GO:0003215] (biological process) Sources: GOC:mtg_heart Definition: The process in which the right cardiac ventricle is generated and organized. Relationships: is a type of cardiac ventricle morphogenesis [GO:0003208]